{
  "term_label": "Unknown molecular function",
  "term_id": "UNKNOWN:0001",
  "gene_symbol": "KCNJ12",
  "gene_name": "ATP-sensitive inward rectifier potassium channel 12",
  "gene": "UniProtKB:Q14500"
}